regulation of vascular endothelial growth factor signaling pathway [GO:1900746] (biological process) Definition: Any process that modulates the frequency, rate or extent of vascular endothelial growth factor signaling pathway. Sources: GOC:TermGenie Also known as: regulation of VEGF signaling, regulation of VEGF-activated signaling pathway, regulation of vascular endothelial growth factor signalling pathway Relationships: is a type of regulation of signal transduction [GO:0009966]; is a type of regulation of cellular response to vascular endothelial growth factor stimulus [GO:1902547]; regulates vascular endothelial growth factor signaling pathway [GO:0038084] Subtypes: negative regulation of vascular endothelial growth factor signaling pathway [GO:1900747], positive regulation of vascular endothelial growth factor signaling pathway [GO:1900748]